{
  "gene_symbol": "TMEM70",
  "term_label": "mitochondrial proton-transporting ATP synthase complex assembly",
  "gene_name": "Transmembrane protein 70, mitochondrial",
  "term_id": "GO:0033615",
  "gene": "UniProtKB:Q9BUB7"
}